{
  "term_label": "negative regulation of T cell activation",
  "term_id": "GO:0050868",
  "gene": "UniProtKB:Q495A1",
  "gene_symbol": "TIGIT",
  "gene_name": "T-cell immunoreceptor with Ig and ITIM domains"
}